{
  "term_id": "GO:0070382",
  "gene_symbol": "UNC13D",
  "gene": "UniProtKB:Q70J99",
  "gene_name": "Protein unc-13 homolog D",
  "term_label": "exocytic vesicle"
}